{
  "gene_name": "Tumor-associated calcium signal transducer 2",
  "term_id": "GO:0005615",
  "term_label": "extracellular space",
  "gene_symbol": "TACSTD2",
  "gene": "UniProtKB:P09758"
}